{
  "term_id": "UNKNOWN:0002",
  "term_label": "Unknown biological process",
  "gene_symbol": "CLCA4",
  "gene_name": "Calcium-activated chloride channel regulator 4",
  "gene": "UniProtKB:Q14CN2"
}